{
  "gene_symbol": "BACE2",
  "gene": "UniProtKB:Q9Y5Z0",
  "gene_name": "Beta-secretase 2",
  "term_label": "plasma membrane",
  "term_id": "GO:0005886"
}